{
  "gene_name": "Proteasome subunit beta type-2",
  "term_id": "GO:0005634",
  "term_label": "nucleus",
  "gene": "UniProtKB:P49721",
  "gene_symbol": "PSMB2"
}